{
  "gene_symbol": "CRYGA",
  "gene": "UniProtKB:P11844",
  "term_id": "GO:0002088",
  "gene_name": "Gamma-crystallin A",
  "term_label": "lens development in camera-type eye"
}